{
  "term_id": "GO:0016020",
  "gene": "UniProtKB:Q969P0",
  "term_label": "membrane",
  "gene_name": "Immunoglobulin superfamily member 8",
  "gene_symbol": "IGSF8"
}